{
  "gene_name": "Calcium-activated potassium channel subunit beta-4",
  "term_id": "GO:0015269",
  "gene": "UniProtKB:Q86W47",
  "gene_symbol": "KCNMB4",
  "term_label": "calcium-activated potassium channel activity"
}